ribbon synapse [GO:0097470] (cellular component) Definition: Type of synapse characterized by an electron-dense ribbon, lamella (bar) or spherical body in the presynaptic process cytoplasm. Subtypes: cochlear hair cell ribbon synapse [GO:0098683], photoreceptor ribbon synapse [GO:0098684] Relationships: is a type of synapse [GO:0045202]; has part synaptic ribbon [GO:0098681] References: PMID:15626493 Sources: NIF_Subcellular:sao1884931180 Also known as: synapsis fasciolaris